{
  "term_label": "transcription coregulator activity",
  "term_id": "GO:0003712",
  "gene_symbol": "AFF4",
  "gene_name": "AF4_FMR2 family member 4",
  "gene": "UniProtKB:Q9UHB7"
}